{
  "term_id": "GO:1990573",
  "gene_name": "ATP-sensitive inward rectifier potassium channel 10",
  "term_label": "potassium ion import across plasma membrane",
  "gene": "UniProtKB:P78508",
  "gene_symbol": "KCNJ10"
}